{
  "gene_name": "Taste receptor type 2 member 31",
  "term_id": "GO:0001580",
  "gene": "UniProtKB:P59538",
  "term_label": "detection of chemical stimulus involved in sensory perception of bitter taste",
  "gene_symbol": "TAS2R31"
}